meiotic mismatch repair involved in meiotic gene conversion [GO:0010776] (biological process) Relationships: is a type of meiotic mismatch repair [GO:0000710]; is part of GO:0006311 Definition: A system for the identification and correction of base-base mismatches, small insertion-deletion loops, and regions of heterology that are present in duplex DNA formed with strands from two recombining molecules resulting in meiotic gene conversion. Meiotic gene conversion is the cell cycle process in which genetic information is transferred from one helix to another. Sources: GOC:dph, GOC:tb